{
  "gene_name": "Reactive oxygen species modulator 1",
  "term_id": "GO:0045039",
  "term_label": "protein insertion into mitochondrial inner membrane",
  "gene": "UniProtKB:P60602",
  "gene_symbol": "ROMO1"
}